{
  "term_label": "cytoplasm",
  "gene": "UniProtKB:Q9HAB8",
  "term_id": "GO:0005737",
  "gene_name": "Phosphopantothenate--cysteine ligase",
  "gene_symbol": "PPCS"
}